{
  "term_label": "intermediate filament organization",
  "gene_name": "Trichohyalin",
  "term_id": "GO:0045109",
  "gene_symbol": "TCHH",
  "gene": "UniProtKB:Q07283"
}